phosphocreatine metabolic process [GO:0006603] (biological process) Definition: The chemical reactions and pathways involving phosphocreatine, a phosphagen of creatine present in high concentration in striated muscle which is synthesized and broken down by creatine phosphokinase to buffer ATP concentration. It acts as an immediate energy reserve for muscle. References: PMID:16371597 Also known as: phosphocreatine metabolism Relationships: is a type of GO:0006575; is a type of phosphate-containing compound metabolic process [GO:0006796]; is a type of GO:0019637 Subtypes: GO:0046314, phosphocreatine catabolic process [GO:0046315]